SCF complex disassembly in response to cadmium stress [GO:1990171] (biological process) Relationships: is a type of protein-containing complex disassembly [GO:0032984]; is part of cellular response to cadmium ion [GO:0071276] References: PMID:23000173 Sources: GOC:rb Definition: The disaggregation of the SCF ubiquitin ligase complex in response to cadmium stress.